{
  "term_label": "Unknown molecular function",
  "gene_name": "Transmembrane protein 50A",
  "gene_symbol": "TMEM50A",
  "gene": "UniProtKB:O95807",
  "term_id": "UNKNOWN:0001"
}